positive regulation of fatty acid oxidation [GO:0046321] (biological process) Also known as: up regulation of fatty acid oxidation, up-regulation of fatty acid oxidation, upregulation of fatty acid oxidation, activation of fatty acid oxidation, stimulation of fatty acid oxidation Relationships: is a type of GO:0045923; is a type of regulation of fatty acid oxidation [GO:0046320]; RO_0002213 fatty acid oxidation [GO:0019395] Definition: Any process that activates or increases the frequency, rate or extent of fatty acid oxidation. Subtypes: positive regulation of fatty acid beta-oxidation [GO:0032000] Sources: GOC:ai